{
  "gene_name": "Cryptic protein",
  "term_label": "anterior/posterior pattern specification",
  "gene": "UniProtKB:P0CG37",
  "term_id": "GO:0009952",
  "gene_symbol": "CFC1"
}